{
  "gene": "UniProtKB:P30559",
  "gene_name": "Oxytocin receptor",
  "term_label": "plasma membrane",
  "gene_symbol": "OXTR",
  "term_id": "GO:0005886"
}